{
  "gene_name": "Nucleoporin NDC1",
  "gene": "UniProtKB:Q9BTX1",
  "term_label": "nuclear pore transmembrane ring",
  "gene_symbol": "NDC1",
  "term_id": "GO:0070762"
}